phosphatidylinositol-3-phosphate biosynthetic process [GO:0036092] (biological process) Definition: The chemical reactions and pathways resulting in the formation of phosphatidylinositol-3-phosphate, a phosphatidylinositol monophosphate carrying the phosphate group at the 3-position. Also known as: PI(3)P biosynthesis, PtdIns3P biosynthesis, phosphatidylinositol-3-phosphate anabolism, phosphatidylinositol-3-phosphate biosynthesis, phosphatidylinositol-3-phosphate formation, phosphatidylinositol-3-phosphate synthesis Relationships: is a type of phosphatidylinositol phosphate biosynthetic process [GO:0046854] Sources: GOC:al, GOC:vw